neuropeptide Y receptor binding [GO:0031841] (molecular function) Definition: Binding to a neuropeptide Y receptor. Relationships: is a type of neuropeptide receptor binding [GO:0071855] Subtypes: GO:0031842, GO:0031843, type 4 neuropeptide Y receptor binding [GO:0031844], type 5 neuropeptide Y receptor binding [GO:0031845] Sources: GOC:mah, GOC:nln Also known as: NPY receptor binding, neuropeptide Y receptor ligand